{
  "gene": "UniProtKB:Q86UT5",
  "term_id": "GO:0016324",
  "term_label": "apical plasma membrane",
  "gene_name": "Na(+)_H(+) exchange regulatory cofactor NHE-RF4",
  "gene_symbol": "NHERF4"
}